PSII associated light-harvesting complex II catabolic process [GO:0010304] (biological process) Also known as: LHCII catabolism Relationships: is a type of protein catabolic process [GO:0030163] Definition: The chemical reactions and pathways resulting in the breakdown of one or more components of the light-harvesting complex of photosystem II. References: PMID:16157880 Sources: GOC:mah Regulation: regulated by regulation of PSII associated light-harvesting complex II catabolic process [GO:0010550]